{
  "gene": "UniProtKB:O75368",
  "term_label": "positive regulation of cytoplasmic translational initiation",
  "gene_symbol": "SH3BGRL",
  "gene_name": "Adapter SH3BGRL",
  "term_id": "GO:1904690"
}